negative regulation of cell junction assembly [GO:1901889] (biological process) Also known as: down regulation of cell junction assembly, down-regulation of cell junction assembly, downregulation of cell junction assembly, inhibition of cell junction assembly Sources: GOC:TermGenie Subtypes: negative regulation of focal adhesion assembly [GO:0051895], GO:0051964, GO:1903347, GO:1903597 Definition: Any process that stops, prevents or reduces the frequency, rate or extent of cell junction assembly. Relationships: is_a negative regulation of cellular component organization [GO:0051129]; is a type of GO:1901888; negatively regulates cell junction assembly [GO:0034329]